mammalian oogenesis stage [GO:0022605] (biological process) Also known as: mammalian oogenesis process Subtypes: GO:0048158, primary oocyte stage [GO:0048159], primary follicle stage [GO:0048160], double layer follicle stage [GO:0048161], multi-layer follicle stage [GO:0048162], scattered antral spaces stage [GO:0048163], distinct antral spaces stage [GO:0048164], GO:0048165, GO:0048166 Sources: GOC:isa_complete, GOC:mtg_sensu Relationships: is a type of multicellular organismal reproductive process [GO:0048609]; is part of oogenesis [GO:0048477] Definition: A reproductive process that is a step in the formation and maturation of an ovum or female gamete from a primordial female germ cell.